negative regulation of NK T cell activation [GO:0051134] (biological process) Definition: Any process that stops, prevents, or reduces the frequency, rate or extent of natural killer T cell activation. References: PMID:12154375, PMID:9133426 Sources: ISBN:0781735149 Also known as: down regulation of NK T cell activation, down-regulation of NK T cell activation, downregulation of NK T cell activation, negative regulation of NK T lymphocyte activation, negative regulation of NK T-cell activation, negative regulation of NK T-lymphocyte activation, negative regulation of NKT cell activation, negative regulation of NT cell activation, negative regulation of natural T cell activation, negative regulation of natural killer T cell activation, inhibition of NK T cell activation Relationships: is a type of negative regulation of alpha-beta T cell activation [GO:0046636]; is a type of regulation of NK T cell activation [GO:0051133]; negatively regulates NK T cell activation [GO:0051132] Subtypes: GO:0051141